{
  "gene_name": "Pleckstrin homology-like domain family A member 2",
  "term_id": "GO:0001890",
  "term_label": "placenta development",
  "gene": "UniProtKB:Q53GA4",
  "gene_symbol": "PHLDA2"
}